regulation of trophectodermal cell proliferation [GO:1904073] (BP) References: PMID:24508636 Sources: GOC:TermGenie, GO_REF:0000058 Definition: Any process that modulates the frequency, rate or extent of trophectodermal cell proliferation. Subtypes: negative regulation of trophectodermal cell proliferation [GO:1904074], positive regulation of trophectodermal cell proliferation [GO:1904075] Also known as: regulation of trophectoderm cell proliferation Relationships: is a type of regulation of cell population proliferation [GO:0042127]; is a type of regulation of developmental growth [GO:0048638]; regulates GO:0001834